termination of mitochondrial transcription [GO:0006393] (BP) Definition: A transcription termination process that completes the production of a primary mitochondrial transcript. References: PMID:29945721 Also known as: RNA transcription termination from mitochondrial promoter, mitochondrial transcription termination Relationships: is a type of mitochondrial RNA metabolic process [GO:0000959]; is a type of DNA-templated transcription termination [GO:0006353]; is part of mitochondrial transcription [GO:0006390]